circadian regulation of systemic arterial blood pressure by hormone [GO:0003067] (BP) Sources: GOC:mtg_cardio Relationships: is a type of GO:0001990; BFO_0000050 GO:0003052 Definition: The process in which hormones modulate the force with which blood passes through the circulatory system contributing to different values of blood pressure oscillating with a regularity of approximately 24 hours. A hormone is one of a group of substances formed in very small amounts in one specialized organ or group of cells and carried (sometimes in the bloodstream) to another organ or group of cells, in the same organism, upon which they have a specific regulatory action.